{
  "gene": "UniProtKB:P05231",
  "term_id": "GO:0005615",
  "gene_name": "Interleukin-6",
  "term_label": "extracellular space",
  "gene_symbol": "IL6"
}